regulation of synaptic plasticity [GO:0048167] (biological process) References: PMID:11891290 Sources: GOC:dph, GOC:jid, GOC:tb Note: Note that the syntax of the definition of this term is different from the usual regulation syntax because it describes regulation of a trait rather than regulation of a process. Relationships: is a type of modulation of chemical synaptic transmission [GO:0050804]; is a type of regulation of biological quality [GO:0065008] Subtypes: negative regulation of synaptic plasticity [GO:0031914], positive regulation of synaptic plasticity [GO:0031915], regulation of synaptic metaplasticity [GO:0031916], regulation of neuronal synaptic plasticity [GO:0048168], regulation of synaptic plasticity by chemical substance [GO:0051913], long-term synaptic potentiation [GO:0060291], long-term synaptic depression [GO:0060292], regulation of synaptic scaling [GO:0150092], regulation of long-term synaptic potentiation [GO:1900271], regulation of long-term synaptic depression [GO:1900452], regulation of short-term synaptic potentiation [GO:1905512], GO:1990926 Definition: A process that modulates synaptic plasticity, the ability of synapses to change as circumstances require. They may alter function, such as increasing or decreasing their sensitivity, or they may increase or decrease in actual numbers.